{
  "term_label": "lysozyme activity",
  "gene_name": "Lysozyme g-like protein 1",
  "gene": "UniProtKB:Q8N1E2",
  "gene_symbol": "LYG1",
  "term_id": "GO:0003796"
}